{
  "gene_symbol": "GIN1",
  "gene": "UniProtKB:Q9NXP7",
  "term_id": "UNKNOWN:0001",
  "gene_name": "Gypsy retrotransposon integrase-like protein 1",
  "term_label": "Unknown molecular function"
}